{
  "gene_name": "Bifunctional peptidase and (3S)-lysyl hydroxylase JMJD7",
  "gene_symbol": "JMJD7",
  "term_label": "Unknown biological process",
  "gene": "UniProtKB:P0C870",
  "term_id": "UNKNOWN:0002"
}